{
  "gene_symbol": "AASS",
  "gene_name": "Alpha-aminoadipic semialdehyde synthase, mitochondrial",
  "term_label": "lysine biosynthetic process via aminoadipic acid",
  "term_id": "GO:0019878",
  "gene": "UniProtKB:Q9UDR5"
}